{
  "gene_name": "LIM domain kinase 1",
  "gene_symbol": "LIMK1",
  "term_id": "GO:0043005",
  "term_label": "neuron projection",
  "gene": "UniProtKB:P53667"
}